pH reduction [GO:0045851] (biological process) Also known as: acidification Sources: GOC:go_curators Definition: Any process that reduces the internal pH of an organism, part of an organism or a cell, measured by the concentration of the hydrogen ion. Relationships: is a type of regulation of pH [GO:0006885]